{
  "term_id": "UNKNOWN:0003",
  "term_label": "Unknown cellular component",
  "gene": "UniProtKB:P35475",
  "gene_name": "Alpha-L-iduronidase",
  "gene_symbol": "IDUA"
}